{
  "gene_symbol": "RYK",
  "gene_name": "Tyrosine-protein kinase RYK",
  "term_label": "Unknown molecular function",
  "term_id": "UNKNOWN:0001",
  "gene": "UniProtKB:P34925"
}